{
  "gene_name": "Microphthalmia-associated transcription factor",
  "term_id": "GO:0030318",
  "term_label": "melanocyte differentiation",
  "gene": "UniProtKB:O75030",
  "gene_symbol": "MITF"
}